antibiotic metabolic process [GO:0016999] (biological process) Subtypes: GO:0017000, antibiotic catabolic process [GO:0017001], macrolide metabolic process [GO:0033067] Sources: GOC:cab2 Also known as: antibiotic metabolism Relationships: is a type of metabolic process [GO:0008152] Definition: The chemical reactions and pathways involving an antibiotic, a substance produced by or derived from certain fungi, bacteria, and other organisms, that can destroy or inhibit the growth of other microorganisms.